{
  "gene": "UniProtKB:Q9UMW8",
  "gene_name": "Ubl carboxyl-terminal hydrolase 18",
  "term_label": "nucleus",
  "gene_symbol": "USP18",
  "term_id": "GO:0005634"
}